{
  "gene": "UniProtKB:O75582",
  "term_id": "GO:0004674",
  "term_label": "protein serine/threonine kinase activity",
  "gene_name": "Ribosomal protein S6 kinase alpha-5",
  "gene_symbol": "RPS6KA5"
}